{
  "gene_name": "Protein S100-A8",
  "term_id": "GO:0043542",
  "term_label": "endothelial cell migration",
  "gene": "UniProtKB:P05109",
  "gene_symbol": "S100A8"
}